UDP-N-acetylglucosamine transmembrane transporter activity [GO:0005462] (molecular function) Definition: Enables the transfer of a UDP-N-acetylglucosamine from one side of a membrane to the other. N-acetylglucosamine is a substance composed of N-acetylglucosamine, a common structural unit of oligosaccharides, in glycosidic linkage with uridine diphosphate. Sources: GOC:ai, GOC:mtg_transport, ISBN:0815340729 Relationships: is a type of pyrimidine nucleotide-sugar transmembrane transporter activity [GO:0015165]; is part of UDP-N-acetylglucosamine transmembrane transport [GO:1990569]